{
  "gene": "UniProtKB:Q8WWR9",
  "gene_symbol": "PPDPFL",
  "term_label": "Unknown biological process",
  "gene_name": "Pancreatic progenitor cell differentiation and proliferation factor-like protein",
  "term_id": "UNKNOWN:0002"
}